primary spermatocyte growth [GO:0007285] (BP) Sources: GOC:jid, ISBN:0879694238 Definition: The phase of growth and gene expression that male germ cells undergo as they enter the spermatocyte stage. The cells grow in volume and transcribe most of the gene products needed for the morphological events that follow meiosis. Relationships: is a type of developmental process involved in reproduction [GO:0003006]; is a type of developmental cell growth [GO:0048588]; BFO_0000050 spermatogenesis [GO:0007283]